{
  "gene": "UniProtKB:A1L3X0",
  "gene_symbol": "ELOVL7",
  "term_label": "fatty acid elongation, polyunsaturated fatty acid",
  "gene_name": "Elongation of very long chain fatty acids protein 7",
  "term_id": "GO:0034626"
}